positive regulation of positive chemotaxis to cAMP [GO:0061122] (biological process) Subtypes: positive regulation of positive chemotaxis to cAMP by chlorinated alkylphenone [GO:0061124] Definition: Any process that increases the rate, frequency, or extent of directed movement of a motile cell or organism up a concentration gradient of 3',5'-cAMP. Relationships: is_a positive regulation of positive chemotaxis [GO:0050927]; is a type of regulation of positive chemotaxis to cAMP [GO:0061118]; positively regulates GO:0043327 Sources: GOC:dph